central nervous system vasculogenesis [GO:0022009] (BP) Sources: GOC:cls, GOC:dgh, GOC:dph, GOC:jid, GO_REF:0000021 Definition: The differentiation of endothelial cells from progenitor cells during blood vessel development, and the de novo formation of blood vessels and tubes in the central nervous system. The capillary endothelial cells in the brain are specialized to form the blood-brain barrier. Relationships: is_a vasculogenesis [GO:0001570]